{
  "term_id": "UNKNOWN:0001",
  "gene": "UniProtKB:P0DPE3",
  "gene_name": "Transmembrane and death domain protein 1",
  "gene_symbol": "TMDD1",
  "term_label": "Unknown molecular function"
}